{
  "gene_symbol": "HS3ST6",
  "gene_name": "Heparan sulfate glucosamine 3-O-sulfotransferase 6",
  "gene": "UniProtKB:Q96QI5",
  "term_id": "UNKNOWN:0003",
  "term_label": "Unknown cellular component"
}